{
  "term_id": "UNKNOWN:0003",
  "term_label": "Unknown cellular component",
  "gene_name": "Transmembrane protein 275",
  "gene_symbol": "TMEM275",
  "gene": "UniProtKB:A0A0U1RQS6"
}